{
  "gene_symbol": "GSK3A",
  "gene": "UniProtKB:P49840",
  "gene_name": "Glycogen synthase kinase-3 alpha",
  "term_id": "GO:0004674",
  "term_label": "protein serine/threonine kinase activity"
}